{
  "gene_name": "Small conductance calcium-activated potassium channel protein 3",
  "term_id": "GO:0005886",
  "gene_symbol": "KCNN3",
  "gene": "UniProtKB:Q9UGI6",
  "term_label": "plasma membrane"
}